rhombomere cell differentiation [GO:0022036] (BP) Relationships: is a type of GO:0030154; is part of GO:0021546 Definition: The process in which a relatively unspecialized cell acquires specialized features of a rhombomere cell. Sources: GOC:cls, GOC:dgh, GOC:dph, GOC:jid, GO_REF:0000021